{
  "gene": "UniProtKB:Q14982",
  "gene_symbol": "OPCML",
  "gene_name": "Opioid-binding protein_cell adhesion molecule",
  "term_id": "GO:0014069",
  "term_label": "postsynaptic density"
}